{
  "term_label": "Unknown molecular function",
  "gene_name": "Uncharacterized protein",
  "gene": "UniProtKB:A0A3B3IRS2",
  "gene_symbol": "LOC647264",
  "term_id": "UNKNOWN:0001"
}